{
  "gene_symbol": "CDC7",
  "gene_name": "Cell division cycle 7-related protein kinase",
  "gene": "UniProtKB:O00311",
  "term_label": "signal transduction",
  "term_id": "GO:0007165"
}